negative regulation of RNA import into nucleus [GO:0046829] (biological process) Definition: Any process that stops, prevents, or reduces the frequency, rate or extent of the movement of RNA from the cytoplasm into the nucleus. Sources: GOC:bf Also known as: down regulation of RNA import into nucleus, down-regulation of RNA import into nucleus, downregulation of RNA import into nucleus, negative regulation of RNA import into cell nucleus, negative regulation of RNA transport from cytoplasm to nucleus, negative regulation of RNA-nucleus import, inhibition of RNA import into nucleus Relationships: is a type of GO:0032240; is a type of GO:0046823; is_a regulation of RNA import into nucleus [GO:0046828]; negatively regulates GO:0006404